{
  "gene_name": "Potassium voltage-gated channel subfamily S member 3",
  "term_id": "GO:0001508",
  "gene": "UniProtKB:Q9BQ31",
  "term_label": "action potential",
  "gene_symbol": "KCNS3"
}